{
  "term_label": "calcium ion transmembrane transport",
  "gene_symbol": "SLC24A3",
  "gene": "UniProtKB:Q9HC58",
  "term_id": "GO:0070588",
  "gene_name": "Sodium_potassium_calcium exchanger 3"
}